{
  "term_id": "GO:0038023",
  "gene": "UniProtKB:Q15399",
  "term_label": "signaling receptor activity",
  "gene_symbol": "TLR1",
  "gene_name": "Toll-like receptor 1"
}